{
  "gene": "UniProtKB:Q0ZGT2",
  "term_id": "GO:0005886",
  "gene_name": "Nexilin",
  "gene_symbol": "NEXN",
  "term_label": "plasma membrane"
}